copper incorporation into copper-sulfur cluster [GO:0018428] (biological process) Definition: The incorporation of copper into a copper-sulfur cluster. Relationships: is a type of GO:0018427 Sources: GOC:ai Also known as: copper incorporation into copper-sulphur cluster